{
  "gene_symbol": "RAET1L",
  "term_label": "natural killer cell mediated cytotoxicity",
  "gene": "UniProtKB:Q5VY80",
  "gene_name": "UL16-binding protein 6",
  "term_id": "GO:0042267"
}